amphisome [GO:0044753] (cellular component) References: PMID:19008921, PMID:9705327 Sources: GOC:autophagy, GOC:sart Definition: Intermediate organelles formed during macroautophagy through the fusion between autophagosomes and endosomes. Relationships: is a type of autophagosome [GO:0005776]